{
  "gene_name": "Ninjurin-1",
  "term_label": "cell-cell adhesion mediator activity",
  "term_id": "GO:0098632",
  "gene_symbol": "NINJ1",
  "gene": "UniProtKB:Q92982"
}